{
  "gene": "UniProtKB:A0A0B4J2F0",
  "term_label": "Unknown molecular function",
  "term_id": "UNKNOWN:0001",
  "gene_symbol": "PIGBOS1",
  "gene_name": "Protein PIGBOS1"
}